{
  "term_label": "Unknown molecular function",
  "gene_symbol": "GMPPA",
  "gene_name": "Mannose-1-phosphate guanyltransferase alpha",
  "gene": "UniProtKB:Q96IJ6",
  "term_id": "UNKNOWN:0001"
}